monocyte migration into blood stream [GO:0035703] (biological process) Definition: The movement of a monocyte from the bone marrow to the blood stream. Also known as: release of monocytes into circulation Sources: CL:0000576, GOC:BHF Relationships: is a type of GO:0071674; is a type of myeloid leukocyte migration [GO:0097529]; is part of blood circulation [GO:0008015]